{
  "term_id": "UNKNOWN:0002",
  "term_label": "Unknown biological process",
  "gene_name": "Thiosulfate:glutathione sulfurtransferase",
  "gene_symbol": "TSTD1",
  "gene": "UniProtKB:Q8NFU3"
}